{
  "term_label": "chromatin remodeling",
  "gene_symbol": "BAZ1B",
  "gene": "UniProtKB:Q9UIG0",
  "gene_name": "Tyrosine-protein kinase BAZ1B",
  "term_id": "GO:0006338"
}